{
  "gene_name": "Dynein axonemal intermediate chain 1",
  "term_label": "outer dynein arm assembly",
  "gene": "UniProtKB:Q9UI46",
  "gene_symbol": "DNAI1",
  "term_id": "GO:0036158"
}